{
  "gene_name": "Teneurin-2",
  "gene": "UniProtKB:Q9NT68",
  "term_label": "protein heterodimerization activity",
  "gene_symbol": "TENM2",
  "term_id": "GO:0046982"
}